{
  "gene_symbol": "LRRK1",
  "term_label": "Unknown cellular component",
  "term_id": "UNKNOWN:0003",
  "gene": "UniProtKB:Q38SD2",
  "gene_name": "Leucine-rich repeat serine_threonine-protein kinase 1"
}